inflorescence morphogenesis [GO:0048281] (biological process) Relationships: is a type of GO:0003006; is a type of shoot system morphogenesis [GO:0010016]; is a type of post-embryonic plant morphogenesis [GO:0090698]; is part of inflorescence development [GO:0010229] Definition: The process in which the anatomical structures of inflorescences are generated and organized. An inflorescence is the part of a seed plant body that is usually above ground and that can bear flowers. Sources: GOC:jid Subtypes: determinate inflorescence morphogenesis [GO:0048282], indeterminate inflorescence morphogenesis [GO:0048283]